positive regulation of synapse maturation [GO:0090129] (biological process) Definition: Any process that increases the extent of synapse maturation, the process that organizes a synapse so that it attains its fully functional state. Relationships: is a type of positive regulation of developmental process [GO:0051094]; is a type of positive regulation of cellular component organization [GO:0051130]; is a type of regulation of synapse maturation [GO:0090128]; positively regulates synapse maturation [GO:0060074] Subtypes: positive regulation of synapse maturation by synaptic transmission [GO:0090127] Sources: GOC:ascb_2009, GOC:dph, GOC:tb